{
  "gene_name": "Immunoglobulin heavy variable 3-72",
  "term_id": "GO:0003823",
  "gene": "UniProtKB:A0A0B4J1Y9",
  "gene_symbol": "IGHV3-72",
  "term_label": "antigen binding"
}